negative regulation of mesonephric glomerulus development [GO:2000088] (biological process) Definition: Any process that stops, prevents, or reduces the frequency, rate or extent of mesonephric glomerulus development. Sources: GOC:mtg_kidney_jan10 Relationships: is a type of negative regulation of glomerulus development [GO:0090194]; is a type of regulation of mesonephric glomerulus development [GO:2000087]; negatively regulates mesonephric glomerulus development [GO:0061224]